{
  "gene_name": "PGC-1 and ERR-induced regulator in muscle protein 1",
  "term_label": "regulation of DNA-templated transcription",
  "gene": "UniProtKB:Q5SV97",
  "term_id": "GO:0006355",
  "gene_symbol": "PERM1"
}